streptomycin biosynthetic process [GO:0019872] (biological process) Also known as: streptomycin anabolism, streptomycin biosynthesis, streptomycin formation, streptomycin synthesis Relationships: is a type of aminoglycoside antibiotic biosynthetic process [GO:0030648]; is a type of polyol biosynthetic process [GO:0046173] Definition: The chemical reactions and pathways resulting in the formation of streptomycin, a commonly used antibiotic in cell culture media; it acts only on prokaryotes and blocks transition from initiation complex to chain elongating ribosome. Sources: GOC:curators